{
  "term_id": "GO:0005615",
  "gene_symbol": "F11",
  "term_label": "extracellular space",
  "gene": "UniProtKB:P03951",
  "gene_name": "Coagulation factor XI"
}